sphinganine-1-phosphate catabolic process [GO:0051874] (biological process) Sources: GOC:ai Relationships: is a type of GO:0006668; is a type of phospholipid catabolic process [GO:0009395]; is a type of GO:0030149 Also known as: dihydrosphingosine-1-phosphate catabolic process, dihydrosphingosine-1-phosphate catabolism Definition: The chemical reactions and pathways resulting in the breakdown of sphinganine-1-phosphate, the phosphorylated derivative of D-erythro-2-amino-1,3-octadecanediol.